{
  "term_label": "branching involved in blood vessel morphogenesis",
  "gene": "UniProtKB:Q7Z6K4",
  "gene_name": "Notch-regulated ankyrin repeat-containing protein",
  "term_id": "GO:0001569",
  "gene_symbol": "NRARP"
}